parthenolide 3beta-hydroxylase activity [GO:0102627] (molecular function) Definition: Catalysis of the reaction: O2 + parthenolide + reduced [NADPH--hemoprotein reductase] = 3beta-hydroxyparthenolide + H+ + H2O + oxidized [NADPH--hemoprotein reductase]. Sources: RHEA:61328 Relationships: is a type of oxidoreductase activity, acting on paired donors, with incorporation or reduction of molecular oxygen, reduced flavin or flavoprotein as one donor, and incorporation of one atom of oxygen [GO:0016712]